{
  "gene_symbol": "FAM110B",
  "gene_name": "Protein FAM110B",
  "term_id": "UNKNOWN:0001",
  "term_label": "Unknown molecular function",
  "gene": "UniProtKB:Q8TC76"
}